{
  "gene": "UniProtKB:Q8N556",
  "gene_symbol": "AFAP1",
  "gene_name": "Actin filament-associated protein 1",
  "term_label": "regulation of signal transduction",
  "term_id": "GO:0009966"
}